{
  "gene": "UniProtKB:Q13829",
  "term_id": "GO:0035024",
  "gene_symbol": "TNFAIP1",
  "gene_name": "BTB_POZ domain-containing adapter for CUL3-mediated RhoA degradation protein 2",
  "term_label": "negative regulation of Rho protein signal transduction"
}